regulation of mesenchymal cell proliferation [GO:0010464] (biological process) Relationships: is_a regulation of cell population proliferation [GO:0042127]; regulates mesenchymal cell proliferation [GO:0010463] Definition: Any process that modulates the frequency, rate or extent of mesenchymal cell proliferation. A mesenchymal cell is a cell that normally gives rise to other cells that are organized as three-dimensional masses, rather than sheets. Sources: GOC:dph, GOC:tb Subtypes: positive regulation of mesenchymal cell proliferation [GO:0002053], regulation of mesenchymal cell proliferation involved in prostate gland development [GO:0060782], regulation of mesenchymal cell proliferation involved in ureter development [GO:0072199], negative regulation of mesenchymal cell proliferation [GO:0072201], regulation of metanephric cap mesenchymal cell proliferation [GO:0090095], regulation of mesenchymal cell proliferation involved in lung development [GO:2000790]